regulation of systemic arterial blood pressure by local renal renin-angiotensin [GO:0003086] (biological process) Sources: GOC:mtg_cardio Relationships: is a type of GO:0003081 Definition: The process in which angiotensinogen metabolites in the kidney modulate the force with which blood passes through the renal circulatory system. The process begins when renin cleaves angiotensinogen.